{
  "gene": "UniProtKB:Q13224",
  "term_label": "excitatory postsynaptic potential",
  "term_id": "GO:0060079",
  "gene_name": "Glutamate receptor ionotropic, NMDA 2B",
  "gene_symbol": "GRIN2B"
}